{
  "term_label": "nucleus",
  "gene_symbol": "ZPR1",
  "gene": "UniProtKB:O75312",
  "gene_name": "Zinc finger protein ZPR1",
  "term_id": "GO:0005634"
}